PSII associated light-harvesting complex II, peripheral complex [GO:0009656] (cellular component) Relationships: is a type of chloroplast thylakoid membrane protein complex [GO:0098807]; is part of PSII associated light-harvesting complex II [GO:0009517] Sources: GOC:lr Definition: Pigment-protein complex primarily associated to PSII in plants, green algae and cyanobacteria. Involved in state transitions that cause migration to PSI under certain environmental conditions such as high light.